host cell postsynaptic membrane [GO:0035792] (CC) Definition: A postsynaptic membrane that is part of a host cell. A postsynaptic membrane is a specialized area of membrane facing the presynaptic membrane on the tip of the nerve ending and separated from it by a minute cleft (the synaptic cleft). Neurotransmitters transmit the signal across the synaptic cleft to the postsynaptic membrane. Sources: GOC:ecd Also known as: other organism post-synaptic membrane, other organism postsynaptic membrane Relationships: is a type of host cell part [GO:0033643]; is part of GO:0033644